L-valine transmembrane transport [GO:1903785] (biological process) Definition: The directed movement of L-valine across a membrane. Relationships: is a type of organic cation transport [GO:0015695]; is_a valine transport [GO:0015829]; is_a L-alpha-amino acid transmembrane transport [GO:1902475] References: PMID:20944394 Sources: GOC:TermGenie, GO_REF:0000069 Subtypes: L-valine transmembrane import into vacuole [GO:0110101], GO:1903805